{
  "gene_name": "Centrosomal AT-AC splicing factor",
  "gene": "UniProtKB:Q86UT8",
  "term_label": "Unknown cellular component",
  "gene_symbol": "CENATAC",
  "term_id": "UNKNOWN:0003"
}